dendritic cell dendrite [GO:0097511] (cellular component) Relationships: is a type of plasma membrane bounded cell projection [GO:0120025] Definition: A branched cellular projection (or cytoplasmic extension) that is extended from the surface of a dendritic immune cell, and which enables the cell to sample luminal pathogens and increase the surface area for antigen presentation to T cells. References: PMID:12200351 Sources: CL:0000451, GOC:BHF, GOC:cjm